{
  "gene_name": "Sulfotransferase 1C4",
  "gene": "UniProtKB:O75897",
  "gene_symbol": "SULT1C4",
  "term_id": "GO:0051923",
  "term_label": "sulfation"
}